cellular response to carbohydrate stimulus [GO:0071322] (biological process) Relationships: is a type of GO:0009743; is a type of cellular response to oxygen-containing compound [GO:1901701] Subtypes: cellular response to disaccharide stimulus [GO:0071324], cellular response to mannitol stimulus [GO:0071325], cellular response to monosaccharide stimulus [GO:0071326], GO:0072709, cellular response to raffinose [GO:0097403] Definition: Any process that results in a change in state or activity of a cell (in terms of movement, secretion, enzyme production, gene expression, etc.) as a result of a carbohydrate stimulus. Sources: GOC:mah